cellodextrin binding [GO:0044584] (molecular function) Definition: Binding to a cellodextrin, a glucose polymer of 2 or more glucose monomers. References: PMID:18952792 Sources: GOC:mengo_curators, GOC:tt Relationships: is a type of polysaccharide binding [GO:0030247]; is a type of GO:0070492